{
  "gene": "UniProtKB:P85298",
  "gene_symbol": "ARHGAP8",
  "gene_name": "Rho GTPase-activating protein 8",
  "term_id": "GO:0005096",
  "term_label": "GTPase activator activity"
}